regulation of plasmatocyte differentiation [GO:0045613] (biological process) Definition: Any process that modulates the frequency, rate or extent of plasmatocyte differentiation. Sources: GOC:go_curators Relationships: is a type of regulation of hemocyte differentiation [GO:0045610]; regulates plasmatocyte differentiation [GO:0042387] Subtypes: GO:0045614, positive regulation of plasmatocyte differentiation [GO:0045615]